long-chain fatty acyl-CoA oxidase activity [GO:0120524] (molecular function) Definition: Catalysis of the reaction: a long-chain 2,3-saturated fatty acyl-CoA + O2 = a long-chain (2E)-enoyl-CoA + H2O2. Sources: RHEA:78851 Note: While there is not universal consensus on the lengths of short-, medium-, long- and very-long-chain fatty acids, the GO uses the definitions in ChEBI (see CHEBI:26666, CHEBI:59554, CHEBI:15904 and CHEBI:27283). Relationships: is a type of acyl-CoA oxidase activity [GO:0003997]